{
  "gene_name": "Interleukin-13",
  "gene": "UniProtKB:P35225",
  "term_id": "GO:0002639",
  "term_label": "positive regulation of immunoglobulin production",
  "gene_symbol": "IL13"
}